{
  "gene_symbol": "A8MX80",
  "gene_name": "Putative UPF0607 protein ENSP00000383144",
  "term_label": "Unknown molecular function",
  "gene": "UniProtKB:A8MX80",
  "term_id": "UNKNOWN:0001"
}